{
  "term_id": "GO:0005615",
  "gene_name": "Chorionic somatomammotropin hormone-like 1",
  "term_label": "extracellular space",
  "gene": "UniProtKB:Q14406",
  "gene_symbol": "CSHL1"
}